{
  "gene_symbol": "IGLV3-22",
  "term_id": "GO:0006955",
  "term_label": "immune response",
  "gene": "UniProtKB:A0A075B6J6",
  "gene_name": "Immunoglobulin lambda variable 3-22"
}